positive regulation of stem cell population maintenance [GO:1902459] (biological process) References: PMID:22969033 Sources: GOC:TermGenie, GOC:hjd Also known as: up regulation of stem cell maintenance, up-regulation of stem cell maintenance, upregulation of stem cell maintenance, activation of stem cell maintenance, activation of maintenance of pluripotency, positive regulation of maintenance of pluripotency, up regulation of maintenance of pluripotency, up-regulation of maintenance of pluripotency, upregulation of maintenance of pluripotency Subtypes: positive regulation of somatic stem cell population maintenance [GO:1904674] Definition: Any process that activates or increases the frequency, rate or extent of stem cell population maintenance. Relationships: is a type of GO:0051094; is a type of GO:0051240; is a type of regulation of stem cell population maintenance [GO:2000036]; positively regulates GO:0019827